{
  "term_id": "UNKNOWN:0001",
  "gene_symbol": "KRTAP10-12",
  "gene_name": "Keratin-associated protein 10-12",
  "gene": "UniProtKB:P60413",
  "term_label": "Unknown molecular function"
}